{
  "gene_symbol": "MMP21",
  "term_label": "collagen catabolic process",
  "gene_name": "Matrix metalloproteinase-21",
  "gene": "UniProtKB:Q8N119",
  "term_id": "GO:0030574"
}